{
  "gene_symbol": "ATP7B",
  "gene": "UniProtKB:P35670",
  "gene_name": "Copper-transporting ATPase 2",
  "term_id": "GO:0005886",
  "term_label": "plasma membrane"
}